{
  "gene_symbol": "ANXA4",
  "term_id": "GO:0001786",
  "gene": "UniProtKB:P09525",
  "term_label": "phosphatidylserine binding",
  "gene_name": "Annexin A4"
}